{
  "gene": "UniProtKB:Q5QFB9",
  "term_id": "UNKNOWN:0002",
  "gene_symbol": "PAPPA-AS1",
  "term_label": "Unknown biological process",
  "gene_name": "Protein PAPPAS"
}